cell surface receptor protein serine/threonine kinase signaling pathway [GO:0007178] (biological process) Sources: GOC:mah, GOC:signaling Definition: The series of molecular signals initiated by an extracellular ligand binding to a receptor on the surface of the target cell where the receptor possesses serine/threonine kinase activity, and ending with the regulation of a downstream cellular process, e.g. transcription. Relationships: is a type of enzyme-linked receptor protein signaling pathway [GO:0007167] Also known as: transmembrane receptor protein serine/threonine kinase signaling pathway, transmembrane receptor protein serine/threonine kinase signalling pathway Subtypes: transforming growth factor beta receptor superfamily signaling pathway [GO:0141091], anti-Mullerian hormone receptor signaling pathway [GO:1990262] Regulation: regulated by regulation of transmembrane receptor protein serine/threonine kinase signaling pathway [GO:0090092]; positively regulated by positive regulation of transmembrane receptor protein serine/threonine kinase signaling pathway [GO:0090100]; RO_0002212 by GO:0090101